{
  "term_label": "Unknown cellular component",
  "gene": "UniProtKB:P0DUD2",
  "gene_symbol": "SPDYE17",
  "term_id": "UNKNOWN:0003",
  "gene_name": "Putative speedy protein E17"
}